{
  "term_id": "GO:0070373",
  "gene": "UniProtKB:Q99956",
  "gene_name": "Dual specificity protein phosphatase 9",
  "gene_symbol": "DUSP9",
  "term_label": "negative regulation of ERK1 and ERK2 cascade"
}